{
  "term_label": "eye development",
  "term_id": "GO:0001654",
  "gene_symbol": "PBX1",
  "gene": "UniProtKB:P40424",
  "gene_name": "Pre-B-cell leukemia transcription factor 1"
}